{
  "term_label": "Unknown molecular function",
  "gene_name": "Brain-enriched guanylate kinase-associated protein",
  "gene": "UniProtKB:Q9BUH8",
  "term_id": "UNKNOWN:0001",
  "gene_symbol": "BEGAIN"
}